{
  "gene_name": "Natural resistance-associated macrophage protein 1",
  "gene": "UniProtKB:P49279",
  "term_label": "endosome membrane",
  "term_id": "GO:0010008",
  "gene_symbol": "SLC11A1"
}